solid phase of interstitial matrix [GO:0140151] (cellular component) Definition: The solid compartment of the interstitial matrix, including interstitial collagens such as fibrillar and fibril-associated collagens and non-collagenous glycoproteins like fibronectin and elastin. References: PMID:3284468, PMID:34807416 Relationships: is a type of external encapsulating structure [GO:0030312]; is part of GO:0005614